{
  "term_label": "cytoplasm",
  "gene_symbol": "KCTD17",
  "gene": "UniProtKB:Q8N5Z5",
  "term_id": "GO:0005737",
  "gene_name": "BTB_POZ domain-containing protein KCTD17"
}